{
  "term_id": "GO:0005634",
  "term_label": "nucleus",
  "gene": "UniProtKB:Q96IF1",
  "gene_symbol": "AJUBA",
  "gene_name": "LIM domain-containing protein ajuba"
}